{
  "term_id": "GO:0019221",
  "gene_name": "Interleukin-12 receptor subunit beta-2",
  "gene": "UniProtKB:Q99665",
  "gene_symbol": "IL12RB2",
  "term_label": "cytokine-mediated signaling pathway"
}